{
  "gene": "UniProtKB:Q9Y2K9",
  "term_id": "GO:0005886",
  "gene_symbol": "STXBP5L",
  "term_label": "plasma membrane",
  "gene_name": "Syntaxin-binding protein 5-like"
}